{
  "gene": "UniProtKB:Q9NQ88",
  "gene_name": "Fructose-2,6-bisphosphatase TIGAR",
  "gene_symbol": "TIGAR",
  "term_label": "cytosol",
  "term_id": "GO:0005829"
}